{
  "gene_symbol": "TRIM51",
  "term_id": "GO:0005737",
  "gene": "UniProtKB:Q9BSJ1",
  "gene_name": "Tripartite motif-containing protein 51",
  "term_label": "cytoplasm"
}